{
  "term_label": "Unknown cellular component",
  "gene": "UniProtKB:P23468",
  "term_id": "UNKNOWN:0003",
  "gene_symbol": "PTPRD",
  "gene_name": "Receptor-type tyrosine-protein phosphatase delta"
}